{
  "gene_symbol": "CHMP1A",
  "gene": "UniProtKB:Q9HD42",
  "term_label": "Unknown molecular function",
  "term_id": "UNKNOWN:0001",
  "gene_name": "Charged multivesicular body protein 1a"
}